{
  "term_label": "DNA-binding transcription factor activity, RNA polymerase II-specific",
  "gene_symbol": "SHOX",
  "term_id": "GO:0000981",
  "gene_name": "Short stature homeobox protein",
  "gene": "UniProtKB:O15266"
}